{
  "term_label": "positive regulation of TOR signaling",
  "gene_name": "Ragulator complex protein LAMTOR2",
  "gene_symbol": "LAMTOR2",
  "term_id": "GO:0032008",
  "gene": "UniProtKB:Q9Y2Q5"
}